negative regulation of inflammatory response [GO:0050728] (biological process) Also known as: anti-inflammatory response, down regulation of inflammatory response, down-regulation of inflammatory response, downregulation of inflammatory response, inhibition of inflammatory response Definition: Any process that stops, prevents, or reduces the frequency, rate or extent of the inflammatory response. Subtypes: negative regulation of acute inflammatory response [GO:0002674], negative regulation of chronic inflammatory response [GO:0002677], negative regulation of inflammatory response to antigenic stimulus [GO:0002862], GO:0035492, GO:0060266, GO:0106015, negative regulation of neuroinflammatory response [GO:0150079], GO:0160028, negative regulation of histamine secretion by mast cell [GO:1903594] Sources: GOC:ai Relationships: is a type of negative regulation of defense response [GO:0031348]; is a type of GO:0032102; is a type of regulation of inflammatory response [GO:0050727]; negatively regulates inflammatory response [GO:0006954]